{
  "term_id": "UNKNOWN:0001",
  "gene": "UniProtKB:Q9BTX3",
  "gene_symbol": "TMEM208",
  "term_label": "Unknown molecular function",
  "gene_name": "Transmembrane protein 208"
}